{
  "gene_name": "Plexin-A1",
  "gene": "UniProtKB:Q9UIW2",
  "gene_symbol": "PLXNA1",
  "term_id": "GO:0071526",
  "term_label": "semaphorin-plexin signaling pathway"
}